{
  "gene": "UniProtKB:O60240",
  "term_label": "lipid catabolic process",
  "term_id": "GO:0016042",
  "gene_name": "Perilipin-1",
  "gene_symbol": "PLIN1"
}